calcium ion transmembrane import into cytosol [GO:0097553] (biological process) Definition: A process in which a calcium ion is transported from one side of a membrane to the other into the cytosol by means of some agent such as a transporter or pore. Subtypes: release of sequestered calcium ion into cytosol [GO:0051209], calcium ion transport into cytosol [GO:0060402], calcium ion import across plasma membrane [GO:0098703] Relationships: is_a calcium ion transmembrane transport [GO:0070588] Also known as: calcium transmembrane import into cytosol, cytosolic calcium ion transport Sources: GOC:vw